{
  "gene_symbol": "GGT2P",
  "term_label": "regulation of immune system process",
  "term_id": "GO:0002682",
  "gene": "UniProtKB:P36268",
  "gene_name": "Inactive glutathione hydrolase 2"
}